Schwann cell chemotaxis [GO:1990751] (biological process) Relationships: is a type of Schwann cell migration [GO:0036135]; is a type of cell chemotaxis [GO:0060326] Regulation: regulated by regulation of Schwann cell chemotaxis [GO:1904266]; negatively regulated by negative regulation of Schwann cell chemotaxis [GO:1904267]; positively regulated by positive regulation of Schwann cell chemotaxis [GO:1904268] Definition: The directed movement of a Schwann cell guided by a specific chemical concentration gradient. Movement may be towards a higher concentration (positive chemotaxis) or towards a lower concentration (negative chemotaxis). References: PMID:16203995